cellular response to type II interferon [GO:0071346] (biological process) Sources: GOC:mah Also known as: cellular response to interferon-gamma, cellular response to type II IFN, cellular response to immune interferon, cellular response to gamma-interferon Definition: Any process that results in a change in state or activity of a cell (in terms of movement, secretion, enzyme production, gene expression, etc.) as a result of an interferon-gamma stimulus. Interferon gamma is the only member of the type II interferon found so far. Relationships: is a type of response to type II interferon [GO:0034341]; is a type of cellular response to cytokine stimulus [GO:0071345]